{
  "gene": "UniProtKB:Q96JK9",
  "gene_symbol": "MAML3",
  "term_label": "nucleoplasm",
  "gene_name": "Mastermind-like protein 3",
  "term_id": "GO:0005654"
}